{
  "term_id": "UNKNOWN:0002",
  "gene_name": "Olfactory receptor 52D1",
  "term_label": "Unknown biological process",
  "gene_symbol": "OR52D1",
  "gene": "UniProtKB:Q9H346"
}